[citrate-(pro-3S)-lyase] thiolesterase activity [GO:0047778] (molecular function) Definition: Catalysis of the reaction: [citrate (pro-3S)-lyase](acetyl form) + H2O = [citrate (pro-3S)-lyase](thiol form) + acetate. Sources: EC:3.1.2.16, MetaCyc:CITRATE-PRO-3S-LYASE-THIOLESTERASE-RXN Relationships: is a type of GO:0016790 Also known as: citrate (pro-3S)-lyase thiolesterase activity, [citrate-(pro-3S)-lyase] thioesterase activity, citrate lyase deacetylase activity, citrate-(pro-3S)-lyase thioesterase activity, citrate-(pro-3S)-lyase thiolesterase activity, citrate-(pro-3S)-lyase(acetyl-form) hydrolase activity